IHF-DNA complex [GO:1990177] (cellular component) References: PMID:17097674 Sources: GOC:bhm Also known as: IHF complex, IHFa-IHFb-DNA complex Definition: A protein-DNA complex containing IHF heterodimers (an alpha and a beta chain) bound to DNA. IHF binds to double-stranded DNA in a structure- and sequence-specific manner and bends the DNA into a nucleosome-like structure, the bacterial nucleoid. Relationships: is a type of protein-DNA complex [GO:0032993]; is_a GO:1990104; is part of bacterial nucleoid [GO:0043590]